{
  "gene_symbol": "SLC27A1",
  "gene_name": "Long-chain fatty acid transport protein 1",
  "gene": "UniProtKB:Q6PCB7",
  "term_label": "long-chain fatty acid metabolic process",
  "term_id": "GO:0001676"
}